{
  "term_label": "cytoplasm",
  "gene_name": "F-box only protein 17",
  "gene_symbol": "FBXO17",
  "term_id": "GO:0005737",
  "gene": "UniProtKB:Q96EF6"
}